{
  "gene_name": "Partitioning defective 3 homolog",
  "term_label": "apical plasma membrane",
  "term_id": "GO:0016324",
  "gene_symbol": "PARD3",
  "gene": "UniProtKB:Q8TEW0"
}